{
  "term_id": "GO:0005484",
  "gene_symbol": "VAMP8",
  "gene": "UniProtKB:Q9BV40",
  "gene_name": "Vesicle-associated membrane protein 8",
  "term_label": "SNAP receptor activity"
}